{
  "term_id": "GO:1902514",
  "gene": "UniProtKB:Q06432",
  "term_label": "regulation of calcium ion transmembrane transport via high voltage-gated calcium channel",
  "gene_name": "Voltage-dependent calcium channel gamma-1 subunit",
  "gene_symbol": "CACNG1"
}